{
  "term_label": "helicase activity",
  "gene": "UniProtKB:Q9H6S0",
  "term_id": "GO:0004386",
  "gene_symbol": "YTHDC2",
  "gene_name": "3'-5' RNA helicase YTHDC2"
}